{
  "gene_symbol": "RCOR3",
  "gene_name": "REST corepressor 3",
  "gene": "UniProtKB:Q9P2K3",
  "term_id": "GO:0045892",
  "term_label": "negative regulation of DNA-templated transcription"
}